{
  "term_label": "mRNA 3'-UTR binding",
  "gene_name": "RNA-binding protein FXR2",
  "gene": "UniProtKB:P51116",
  "gene_symbol": "FXR2",
  "term_id": "GO:0003730"
}